{
  "term_label": "Unknown molecular function",
  "gene_name": "Proline-rich protein PRCC",
  "term_id": "UNKNOWN:0001",
  "gene_symbol": "PRCC",
  "gene": "UniProtKB:Q92733"
}